{
  "gene_symbol": "POF1B",
  "term_id": "GO:0051015",
  "gene_name": "Protein POF1B",
  "gene": "UniProtKB:Q8WVV4",
  "term_label": "actin filament binding"
}